{
  "gene_name": "Probable cation-transporting ATPase 13A4",
  "gene": "UniProtKB:Q4VNC1",
  "term_label": "ATPase-coupled monoatomic cation transmembrane transporter activity",
  "term_id": "GO:0019829",
  "gene_symbol": "ATP13A4"
}